{
  "gene_symbol": "SLC30A4",
  "gene_name": "Probable proton-coupled zinc antiporter SLC30A4",
  "gene": "UniProtKB:O14863",
  "term_id": "GO:0010043",
  "term_label": "response to zinc ion"
}